miRNA-mediated gene silencing by inhibition of translation [GO:0035278] (biological process) References: PMID:14744438, PMID:15196554 Also known as: down regulation of translation involved in gene silencing by miRNA, down-regulation of translation involved in gene silencing by miRNA, downregulation of translation involved in gene silencing by miRNA, gene silencing by miRNA, negative regulation of translation, miRNA mediated inhibition of translation, negative regulation of translation involved in gene silencing by microRNA, inhibition of translation involved in gene silencing by miRNA, miRNA-mediated gene silencing, negative regulation of translation Relationships: is a type of negative regulation of translation [GO:0017148]; is_a GO:0035195 Definition: An RNA interference pathway in which microRNAs (miRNAs) block the translation of target mRNAs into proteins. Once incorporated into a RNA-induced silencing complex (RISC), a miRNA will typically mediate repression of translation if the miRNA imperfectly base-pairs with the 3' untranslated regions of target mRNAs.